{
  "term_label": "ERAD pathway",
  "term_id": "GO:0036503",
  "gene_name": "Ubiquitin-conjugating enzyme E2 J2",
  "gene_symbol": "UBE2J2",
  "gene": "UniProtKB:Q8N2K1"
}